negative regulation of membrane depolarization during AV node cell action potential [GO:1905028] (biological process) Also known as: down regulation of membrane depolarization during AV node cardiac muscle cell action potential, down regulation of membrane depolarization during AV node cell action potential, down regulation of membrane depolarization during atrioventricular node cardiac muscle cell action potential, down-regulation of membrane depolarization during AV node cardiac muscle cell action potential, down-regulation of membrane depolarization during AV node cell action potential, down-regulation of membrane depolarization during atrioventricular node cardiac muscle cell action potential, downregulation of membrane depolarization during AV node cardiac muscle cell action potential, downregulation of membrane depolarization during AV node cell action potential, downregulation of membrane depolarization during atrioventricular node cardiac muscle cell action potential, negative regulation of membrane depolarization during AV node cardiac muscle cell action potential, negative regulation of membrane depolarization during atrioventricular node cardiac muscle cell action potential, inhibition of membrane depolarization during AV node cardiac muscle cell action potential, inhibition of membrane depolarization during AV node cell action potential, inhibition of membrane depolarization during atrioventricular node cardiac muscle cell action potential Definition: Any process that stops, prevents or reduces the frequency, rate or extent of membrane depolarization during AV node cell action potential. Relationships: is a type of negative regulation of membrane depolarization during cardiac muscle cell action potential [GO:1900826]; is a type of GO:1905027; negatively regulates membrane depolarization during AV node cell action potential [GO:0086045] References: PMID:19726871 Sources: GOC:BHF, GOC:BHF_miRNA, GOC:TermGenie, GOC:mtg_cardiac_conduct_nov11, GOC:rph